{
  "gene_name": "Ran-binding protein 6",
  "term_label": "cytoplasm",
  "gene_symbol": "RANBP6",
  "gene": "UniProtKB:O60518",
  "term_id": "GO:0005737"
}